{
  "gene_name": "Olfactory receptor 6C6",
  "gene_symbol": "OR6C6",
  "gene": "UniProtKB:A6NF89",
  "term_id": "GO:0004984",
  "term_label": "olfactory receptor activity"
}